{
  "gene_name": "GTP-binding protein Di-Ras1",
  "gene_symbol": "DIRAS1",
  "gene": "UniProtKB:O95057",
  "term_label": "plasma membrane",
  "term_id": "GO:0005886"
}